response to camptothecin [GO:1901563] (biological process) Definition: Any process that results in a change in state or activity of a cell or an organism (in terms of movement, secretion, enzyme production, gene expression, etc.) as a result of a camptothecin stimulus. Subtypes: cellular response to camptothecin [GO:0072757] Sources: GOC:TermGenie Relationships: is_a response to alkaloid [GO:0043279]; is a type of GO:0097305 Also known as: response to CPT